purine ribonucleoside triphosphate biosynthetic process [GO:0009206] (biological process) Relationships: is a type of purine nucleoside triphosphate biosynthetic process [GO:0009145]; is a type of ribonucleoside triphosphate biosynthetic process [GO:0009201]; is a type of GO:0009205 Sources: GOC:go_curators, ISBN:0198506732 Also known as: purine ribonucleoside triphosphate anabolism, purine ribonucleoside triphosphate biosynthesis, purine ribonucleoside triphosphate formation, purine ribonucleoside triphosphate synthesis Definition: The chemical reactions and pathways resulting in the formation of purine ribonucleoside triphosphate, a compound consisting of a purine base linked to a ribose sugar esterified with triphosphate on the sugar. Subtypes: GTP biosynthetic process [GO:0006183], ATP biosynthetic process [GO:0006754], GO:0046042